syntaxin-6-syntaxin-16-Vti1a complex [GO:0070067] (cellular component) Relationships: is a type of SNARE complex [GO:0031201] References: PMID:11839770 Definition: A SNARE complex that contains syntaxin 6, syntaxin 16, and Vti1a (or orthologs thereof).